{
  "gene_name": "Epiplakin",
  "term_label": "keratin filament binding",
  "gene_symbol": "EPPK1",
  "gene": "UniProtKB:P58107",
  "term_id": "GO:1990254"
}